{
  "term_label": "neuropeptide signaling pathway",
  "gene": "UniProtKB:Q13519",
  "gene_symbol": "PNOC",
  "term_id": "GO:0007218",
  "gene_name": "Prepronociceptin"
}